{
  "gene_name": "Dolichyl-diphosphooligosaccharide--protein glycosyltransferase 48 kDa subunit",
  "term_id": "GO:0018279",
  "gene_symbol": "DDOST",
  "gene": "UniProtKB:P39656",
  "term_label": "protein N-linked glycosylation via asparagine"
}